{
  "term_label": "Unknown molecular function",
  "gene": "UniProtKB:Q4G0W2",
  "gene_symbol": "DUSP28",
  "gene_name": "Dual specificity phosphatase 28",
  "term_id": "UNKNOWN:0001"
}